{
  "term_label": "catenin complex",
  "gene_symbol": "CDH23",
  "gene_name": "Cadherin-23",
  "gene": "UniProtKB:Q9H251",
  "term_id": "GO:0016342"
}